{
  "term_id": "GO:0005765",
  "term_label": "lysosomal membrane",
  "gene_symbol": "TMEM79",
  "gene_name": "Transmembrane protein 79",
  "gene": "UniProtKB:Q9BSE2"
}